protein localization to Cajal body [GO:1904867] (biological process) Definition: A process in which a protein is transported to, or maintained in, a location within a Cajal body. References: PMID:25467444 Sources: GOC:BHF, GOC:BHF_telomere, GOC:TermGenie, GOC:nc, GO_REF:0000087 Also known as: protein localisation in Cajal body, protein localisation to Cajal body, protein localization in Cajal body Relationships: is a type of protein localization to nuclear body [GO:1903405] Regulation: regulated by regulation of protein localization to Cajal body [GO:1904869]; negatively regulated by negative regulation of protein localization to Cajal body [GO:1904870]; positively regulated by positive regulation of protein localization to Cajal body [GO:1904871]